{
  "gene_symbol": "KRTAP5-11",
  "gene_name": "Keratin-associated protein 5-11",
  "term_id": "UNKNOWN:0001",
  "term_label": "Unknown molecular function",
  "gene": "UniProtKB:Q6L8G4"
}